malate transmembrane transporter activity [GO:0015140] (molecular function) Relationships: is_a GO:0005310; is a type of C4-dicarboxylate transmembrane transporter activity [GO:0015556]; is part of GO:0071423 Also known as: dicarboxylate (succinate/fumarate/malate) antiporter activity Definition: Enables the transfer of malate from one side of a membrane to the other. Malate is a chiral hydroxydicarboxylic acid, hydroxybutanedioic acid. The (+) enantiomer is an important intermediate in metabolism as a component of both the TCA cycle and the glyoxylate cycle. Sources: GOC:ai Subtypes: GO:0015366, oxoglutarate:malate antiporter activity [GO:0015367], malate:sodium symporter activity [GO:0043882]